etioplast envelope [GO:0034425] (cellular component) Definition: The double lipid bilayer enclosing the etioplast and separating its contents from the rest of the cytoplasm; includes the intermembrane space. Sources: GOC:mah Relationships: is a type of plastid envelope [GO:0009526]; BFO_0000050 etioplast [GO:0009513]